pyrimidine nucleotide-sugar transmembrane transport [GO:0090481] (biological process) Relationships: is a type of nucleotide-sugar transmembrane transport [GO:0015780] Subtypes: CMP-N-acetylneuraminate transmembrane transport [GO:0015782], UDP-glucose transmembrane transport [GO:0015786], UDP-glucuronate transmembrane transport [GO:0015787], UDP-N-acetylgalactosamine transmembrane transport [GO:0015789], UDP-xylose transmembrane transport [GO:0015790], GO:0072334, GO:0140821, UDP-N-acetylglucosamine transmembrane transport [GO:1990569] Also known as: pyrimidine nucleotide-sugar membrane transport, pyrimidine nucleotide-sugar transport Sources: GOC:tb Definition: The process in which a pyrimidine nucleotide-sugar is transported across a membrane. Pyrimidine nucleotide-sugars are pyrimidine nucleotides in glycosidic linkage with a monosaccharide or monosaccharide derivative. Note: Note that this term is not intended for use in annotating lateral movement within membranes.